serine import into mitochondrion [GO:0140300] (biological process) References: PMID:30442778 Definition: The process in which serine is transported from the cytosol into the mitochondrial matrix. Relationships: is a type of amino acid transmembrane transport [GO:0003333]; is a type of serine transport [GO:0032329]; is a type of import into the mitochondrion [GO:0170036]; is a type of carboxylic acid transmembrane transport [GO:1905039]